{
  "gene_name": "P antigen family member 5",
  "gene_symbol": "PAGE5",
  "gene": "UniProtKB:Q96GU1",
  "term_id": "UNKNOWN:0001",
  "term_label": "Unknown molecular function"
}